{
  "gene_symbol": "USP20",
  "term_label": "nervous system development",
  "gene": "UniProtKB:Q9Y2K6",
  "term_id": "GO:0007399",
  "gene_name": "Ubiquitin carboxyl-terminal hydrolase 20"
}